negative regulation of defense response to virus [GO:0050687] (biological process) Sources: GOC:ai Subtypes: negative regulation of defense response to virus by host [GO:0050689] Also known as: down regulation of antiviral response, down-regulation of antiviral response, downregulation of antiviral response, negative regulation of antiviral response, inhibition of antiviral response Relationships: is a type of negative regulation of response to biotic stimulus [GO:0002832]; is a type of negative regulation of defense response [GO:0031348]; is a type of negative regulation of response to external stimulus [GO:0032102]; is a type of regulation of defense response to virus [GO:0050688]; negatively regulates defense response to virus [GO:0051607] Definition: Any process that stops, prevents or reduces the rate or extent of antiviral mechanisms, thereby facilitating viral replication.